G-quadruplex DNA binding [GO:0051880] (molecular function) Subtypes: telomeric G-quadruplex DNA binding [GO:0061849] References: PMID:16142245, PMID:9512530 Definition: Binding to G-quadruplex DNA structures, in which groups of four guanines adopt a flat, cyclic Hoogsteen hydrogen-bonding arrangement known as a guanine tetrad. The stacking of guanine tetrads results in G-quadruplex DNA structures. G-quadruplex DNA can form under physiological conditions from some G-rich sequences, such as those found in telomeres, immunoglobulin switch regions, gene promoters, fragile X repeats, and the dimerization domain in the human immunodeficiency virus (HIV) genome. Relationships: is a type of DNA binding [GO:0003677] Also known as: G quartet binding, G-quartet binding, G quadruplex DNA binding, G quartet DNA binding, G-DNA binding, G-quartet DNA binding, quadruplex DNA binding, tetraplex DNA binding